{
  "gene": "UniProtKB:O95749",
  "term_id": "GO:0004311",
  "gene_symbol": "GGPS1",
  "term_label": "geranylgeranyl diphosphate synthase activity",
  "gene_name": "Geranylgeranyl pyrophosphate synthase"
}